magnesium ion homeostasis [GO:0010960] (biological process) Subtypes: intracellular magnesium ion homeostasis [GO:0010961] Relationships: is a type of GO:0055080; is a type of inorganic ion homeostasis [GO:0098771] Definition: Any process involved in the maintenance of an internal steady state of magnesium ions within an organism or cell. Sources: GOC:dph, GOC:tb